{
  "gene": "UniProtKB:Q5VTQ0",
  "gene_symbol": "TTC39B",
  "term_label": "negative regulation of cholesterol storage",
  "gene_name": "Tetratricopeptide repeat protein 39B",
  "term_id": "GO:0010887"
}